galactolipid catabolic process [GO:0019376] (biological process) Subtypes: galactosylceramide catabolic process [GO:0006683] Also known as: galactolipid breakdown, galactolipid catabolism, galactolipid degradation Sources: ISBN:0198506732 Definition: The chemical reactions and pathways resulting in the breakdown of galactolipids, any glycolipid containing one of more residues of galactose and/or N-acetylgalactosamine. Relationships: is a type of GO:0019374; is a type of glycolipid catabolic process [GO:0019377]